{
  "gene_name": "Interferon omega-1",
  "gene": "UniProtKB:P05000",
  "gene_symbol": "IFNW1",
  "term_label": "extracellular space",
  "term_id": "GO:0005615"
}